{
  "term_label": "GTPase activity",
  "gene": "UniProtKB:P11488",
  "gene_name": "Guanine nucleotide-binding protein G(t) subunit alpha-1",
  "term_id": "GO:0003924",
  "gene_symbol": "GNAT1"
}